extracellular matrix constituent secretion [GO:0070278] (biological process) Regulation: regulated by regulation of extracellular matrix constituent secretion [GO:0003330]; positively regulated by positive regulation of extracellular matrix constituent secretion [GO:0003331]; negatively regulated by negative regulation of extracellular matrix constituent secretion [GO:0003332] Relationships: is_a secretion by cell [GO:0032940]; BFO_0000050 GO:0030198 Also known as: ECM constituent secretion, ECM secretion Subtypes: basement membrane constituent secretion [GO:0061864], dentin extracellular matrix secretion [GO:0070468] Sources: GOC:mah Definition: The controlled release of molecules that form the extracellular matrix, including carbohydrates and glycoproteins by a cell.